{
  "gene_name": "M-phase inducer phosphatase 2",
  "term_label": "positive regulation of G2/M transition of mitotic cell cycle",
  "gene": "UniProtKB:P30305",
  "term_id": "GO:0010971",
  "gene_symbol": "CDC25B"
}